{
  "gene_symbol": "H2BC18",
  "term_label": "innate immune response in mucosa",
  "gene": "UniProtKB:Q5QNW6",
  "term_id": "GO:0002227",
  "gene_name": "Histone H2B type 2-F"
}